{
  "term_label": "translation factor activity, RNA binding",
  "term_id": "GO:0008135",
  "gene_symbol": "CPEB4",
  "gene_name": "Cytoplasmic polyadenylation element-binding protein 4",
  "gene": "UniProtKB:Q17RY0"
}